{
  "gene_name": "Sodium channel protein type 3 subunit alpha",
  "gene": "UniProtKB:Q9NY46",
  "term_label": "sodium ion transmembrane transport",
  "gene_symbol": "SCN3A",
  "term_id": "GO:0035725"
}